histone H3 arginine deiminase activity [GO:0141057] (molecular function) Definition: Catalysis of the reaction: H2O + histone H3 L-arginyl = histone H3 L-citrullyl + NH4+, resulting in histone H3 citrullination. References: PMID:25303536 Relationships: is a type of GO:0140794 Subtypes: histone H3R2 arginine deiminase activity [GO:0140795], GO:0140796, histone H3R17 arginine deiminase activity [GO:0140797], histone H3R26 arginine deiminase activity [GO:0140798]